{
  "gene_symbol": "KDR",
  "term_label": "cell surface receptor protein tyrosine kinase signaling pathway",
  "term_id": "GO:0007169",
  "gene": "UniProtKB:P35968",
  "gene_name": "Vascular endothelial growth factor receptor 2"
}